centromere clustering [GO:0098653] (biological process) Definition: The process by which centromeres/kinetochores become localized to clusters. Also known as: kinetochore clustering References: PMID:10761928, PMID:23283988, PMID:8486732 Sources: GOC:di, GOC:dos Subtypes: centromere clustering at the mitotic interphase nuclear envelope [GO:0072766], meiotic centromere clustering [GO:1990571] Note: As inner kinetochores are an integral part of centromeres, we treat centromere and kinetochore clustering as the same process. Relationships: is a type of chromosome localization [GO:0050000]; is a type of centromere localization [GO:0072765]